positive regulation of telomere maintenance in response to DNA damage [GO:1904507] (biological process) Relationships: is a type of positive regulation of telomere maintenance [GO:0032206]; is a type of positive regulation of response to stimulus [GO:0048584]; is a type of regulation of telomere maintenance in response to DNA damage [GO:1904505]; positively regulates telomere maintenance in response to DNA damage [GO:0043247] Subtypes: positive regulation of protection from non-homologous end joining at telomere [GO:1905766] Definition: Any process that activates or increases the frequency, rate or extent of telomere maintenance in response to DNA damage. References: PMID:22579284 Sources: GOC:BHF, GOC:BHF_telomere, GOC:TermGenie, GOC:nc, GO_REF:0000058 Also known as: positive regulation of DNA damage response, telomere maintenance, up regulation of DNA damage response, telomere maintenance, up regulation of telomere maintenance in response to DNA damage, up-regulation of DNA damage response, telomere maintenance, up-regulation of telomere maintenance in response to DNA damage, upregulation of DNA damage response, telomere maintenance, upregulation of telomere maintenance in response to DNA damage, activation of DNA damage response, telomere maintenance, activation of telomere maintenance in response to DNA damage